{
  "gene_symbol": "MCTP2",
  "gene": "UniProtKB:Q6DN12",
  "term_id": "GO:0005509",
  "gene_name": "Multiple C2 and transmembrane domain-containing protein 2",
  "term_label": "calcium ion binding"
}